{
  "term_label": "stearoyl-CoA 9-desaturase activity",
  "gene_name": "Stearoyl-CoA desaturase",
  "term_id": "GO:0004768",
  "gene": "UniProtKB:O00767",
  "gene_symbol": "SCD"
}